{
  "gene_symbol": "FDX1",
  "gene_name": "Adrenodoxin, mitochondrial",
  "gene": "UniProtKB:P10109",
  "term_label": "electron transfer activity",
  "term_id": "GO:0009055"
}